{
  "gene_symbol": "IFT88",
  "term_id": "GO:0042073",
  "term_label": "intraciliary transport",
  "gene_name": "Intraflagellar transport protein 88 homolog",
  "gene": "UniProtKB:Q13099"
}